{
  "term_id": "GO:0005886",
  "term_label": "plasma membrane",
  "gene_symbol": "PTGER1",
  "gene_name": "Prostaglandin E2 receptor EP1 subtype",
  "gene": "UniProtKB:P34995"
}